{
  "gene": "UniProtKB:P30556",
  "term_label": "regulation of blood pressure",
  "gene_name": "Type-1 angiotensin II receptor",
  "gene_symbol": "AGTR1",
  "term_id": "GO:0008217"
}